signal recognition particle [GO:0048500] (cellular component) Subtypes: GO:0005786, signal recognition particle, plasma membrane targeting [GO:0048501], signal recognition particle, chloroplast targeting [GO:0080085] Definition: A complex of protein and RNA which facilitates translocation of proteins across membranes. Relationships: is a type of ribonucleoprotein complex [GO:1990904]; BFO_0000050 cytoplasm [GO:0005737] Sources: GOC:mlg